3-chloroacrylic acid metabolic process [GO:0018888] (biological process) Relationships: is_a monocarboxylic acid metabolic process [GO:0032787]; is_a organohalogen metabolic process [GO:0090345] Definition: The chemical reactions and pathways involving 3-chloroacrylic acid, ClHC=CHCOOH, a chlorinated derivative of acrylic acid. Also known as: 3-chloroacrylic acid metabolism Sources: GOC:ai